{
  "gene_symbol": "KIF21A",
  "gene_name": "Kinesin-like protein KIF21A",
  "gene": "UniProtKB:Q7Z4S6",
  "term_id": "GO:0007018",
  "term_label": "microtubule-based movement"
}